{
  "term_label": "Unknown molecular function",
  "gene": "UniProtKB:P19876",
  "term_id": "UNKNOWN:0001",
  "gene_name": "C-X-C motif chemokine 3",
  "gene_symbol": "CXCL3"
}